{
  "gene_name": "Interferon-inducible protein AIM2",
  "term_label": "nucleoplasm",
  "term_id": "GO:0005654",
  "gene": "UniProtKB:O14862",
  "gene_symbol": "AIM2"
}